ERBB2-ERBB3 signaling pathway [GO:0038133] (biological process) Also known as: ERBB2-ERBB3 signalling pathway, HER2-HER3 signaling pathway Relationships: is a type of GO:0038128; is a type of ERBB3 signaling pathway [GO:0038129] References: PMID:16460914 Sources: GOC:signaling Definition: The series of molecular signals initiated by binding of a ligand to a ERBB3 receptor on the surface of a cell, followed by transmission of the signal by a heterodimeric complex of ERBB2 and ERBB3. ERBB2, which does not bind any known ligand, is activated through formation of a heterodimer with another ligand-activated ERBB family member such as ERBB3. ERBB3 also has impaired kinase activity and relies on ERBB2 for activation and signal transmission.